ubiquitin ligase activator activity [GO:1990757] (molecular function) Definition: Binds to and increases the activity of a ubiquitin ligase. Also known as: mitotic anaphase-promoting complex activator activity Relationships: is a type of ubiquitin-protein transferase activator activity [GO:0097027]; is part of positive regulation of ubiquitin protein ligase activity [GO:1904668] References: PMID:25619242 Sources: GOC:dph